primary cell wall [GO:0009530] (cellular component) References: PMID:9442872 Sources: GOC:jid Relationships: is a type of plant-type cell wall [GO:0009505] Definition: A plant cell wall that is still able to expand, permitting cell growth. Primary cell walls contain more pectin than secondary walls and no lignin is present.